{
  "gene_symbol": "HYAL3",
  "gene_name": "Hyaluronidase-3",
  "term_id": "GO:0001669",
  "gene": "UniProtKB:O43820",
  "term_label": "acrosomal vesicle"
}